{
  "gene_symbol": "SYT2",
  "term_label": "calcium-dependent activation of synaptic vesicle fusion",
  "gene_name": "Synaptotagmin-2",
  "term_id": "GO:0099502",
  "gene": "UniProtKB:Q8N9I0"
}